{
  "gene_symbol": "PHB1",
  "gene_name": "Prohibitin 1",
  "gene": "UniProtKB:P35232",
  "term_label": "mitochondrion",
  "term_id": "GO:0005739"
}